{
  "gene_name": "NF-kappa-B inhibitor-interacting Ras-like protein 1",
  "gene_symbol": "NKIRAS1",
  "gene": "UniProtKB:Q9NYS0",
  "term_label": "GTPase activating protein binding",
  "term_id": "GO:0032794"
}